{
  "term_label": "retinol metabolic process",
  "gene_symbol": "LRAT",
  "gene_name": "Lecithin retinol acyltransferase",
  "term_id": "GO:0042572",
  "gene": "UniProtKB:O95237"
}